{
  "term_label": "neuropeptide binding",
  "gene_name": "Somatostatin receptor type 4",
  "term_id": "GO:0042923",
  "gene_symbol": "SSTR4",
  "gene": "UniProtKB:P31391"
}